{
  "term_id": "UNKNOWN:0003",
  "term_label": "Unknown cellular component",
  "gene_name": "Major facilitator superfamily domain-containing protein 9",
  "gene": "UniProtKB:Q8NBP5",
  "gene_symbol": "MFSD9"
}